{
  "gene": "UniProtKB:Q9Y2Q9",
  "term_label": "Unknown molecular function",
  "term_id": "UNKNOWN:0001",
  "gene_symbol": "MRPS28",
  "gene_name": "Small ribosomal subunit protein bS1m"
}